{
  "gene_name": "Zinc finger protein 624",
  "gene": "UniProtKB:Q9P2J8",
  "gene_symbol": "ZNF624",
  "term_id": "GO:0000978",
  "term_label": "RNA polymerase II cis-regulatory region sequence-specific DNA binding"
}